{
  "gene": "UniProtKB:P35670",
  "gene_symbol": "ATP7B",
  "gene_name": "Copper-transporting ATPase 2",
  "term_id": "GO:0060003",
  "term_label": "copper ion export"
}